{
  "term_id": "GO:0055085",
  "gene_symbol": "ABCB5",
  "gene": "UniProtKB:Q2M3G0",
  "gene_name": "ATP-binding cassette sub-family B member 5",
  "term_label": "transmembrane transport"
}